regulation of heparan sulfate proteoglycan biosynthetic process [GO:0010908] (biological process) Sources: GOC:curators Definition: Any process that modulates the rate, frequency or extent of heparan sulfate proteoglycan biosynthesis. Heparan sulfate proteoglycan biosynthetic processes are the chemical reactions and pathways resulting in the formation of the heparan sulfate proteoglycan, which consists of a core protein linked to a heparan sulfate glycosaminoglycan. The heparan sulfate chain is composed of the repeating disaccharide unit beta-(1,4)-N-acetyl-D-glucosamine-alpha-(1,4)-hexuronic acid. Relationships: is a type of GO:1904098; regulates heparan sulfate proteoglycan biosynthetic process [GO:0015012] Subtypes: positive regulation of heparan sulfate proteoglycan biosynthetic process [GO:0010909]